{
  "term_label": "chloride:bicarbonate antiporter activity",
  "term_id": "GO:0140900",
  "gene_name": "Sulfate transporter",
  "gene": "UniProtKB:P50443",
  "gene_symbol": "SLC26A2"
}